{
  "gene_symbol": "RPP21",
  "term_id": "GO:0008033",
  "term_label": "tRNA processing",
  "gene_name": "Ribonuclease P protein subunit p21",
  "gene": "UniProtKB:Q9H633"
}